{
  "gene_name": "1,5-anhydro-D-fructose reductase",
  "term_id": "GO:0005829",
  "term_label": "cytosol",
  "gene": "UniProtKB:Q96JD6",
  "gene_symbol": "AKR1E2"
}